{
  "term_id": "UNKNOWN:0001",
  "term_label": "Unknown molecular function",
  "gene_symbol": "PDCD2L",
  "gene_name": "Programmed cell death protein 2-like",
  "gene": "UniProtKB:Q9BRP1"
}